nitric oxide sensor activity [GO:0035991] (molecular function) Definition: Binding to and responding, e.g. by conformational change, to changes in the cellular level of nitric oxide (NO). References: PMID:21491957 Sources: GOC:kmv Also known as: NO sensor activity Relationships: is a type of molecular sensor activity [GO:0140299]; is part of response to nitric oxide [GO:0071731]; has part nitric oxide binding [GO:0070026]